{
  "term_id": "UNKNOWN:0003",
  "gene": "UniProtKB:P39877",
  "term_label": "Unknown cellular component",
  "gene_name": "Phospholipase A2 group V",
  "gene_symbol": "PLA2G5"
}